{
  "term_id": "GO:0071013",
  "gene": "UniProtKB:P63162",
  "term_label": "catalytic step 2 spliceosome",
  "gene_name": "Small nuclear ribonucleoprotein-associated protein N",
  "gene_symbol": "SNRPN"
}